triose phosphate transport [GO:0015717] (biological process) Also known as: aldotriose phosphate transport Subtypes: triose phosphate transmembrane transport [GO:0035436] Definition: The directed movement of triose phosphate into, out of or within a cell, or between cells, by means of some agent such as a transporter or pore. Sources: GOC:krc Relationships: is a type of GO:0015748; is a type of carbohydrate derivative transport [GO:1901264]